{
  "gene_name": "C-C motif chemokine 4",
  "gene_symbol": "CCL4",
  "term_label": "inflammatory response",
  "term_id": "GO:0006954",
  "gene": "UniProtKB:P13236"
}